{
  "term_id": "GO:0005737",
  "gene": "UniProtKB:Q9Y536",
  "gene_symbol": "PPIAL4A",
  "term_label": "cytoplasm",
  "gene_name": "Peptidyl-prolyl cis-trans isomerase A-like 4A"
}